{
  "gene_name": "Protein Smaug homolog 1",
  "term_id": "GO:0000932",
  "gene": "UniProtKB:Q9UPU9",
  "term_label": "P-body",
  "gene_symbol": "SAMD4A"
}